{
  "gene": "UniProtKB:O75382",
  "gene_symbol": "TRIM3",
  "term_id": "UNKNOWN:0003",
  "term_label": "Unknown cellular component",
  "gene_name": "Tripartite motif-containing protein 3"
}